{
  "gene_symbol": "LPAR5",
  "gene": "UniProtKB:Q9H1C0",
  "term_label": "behavioral response to pain",
  "gene_name": "Lysophosphatidic acid receptor 5",
  "term_id": "GO:0048266"
}